{
  "gene": "UniProtKB:Q16719",
  "term_id": "GO:0043420",
  "gene_symbol": "KYNU",
  "gene_name": "Kynureninase",
  "term_label": "anthranilate metabolic process"
}